{
  "gene": "UniProtKB:P37840",
  "gene_symbol": "SNCA",
  "gene_name": "Alpha-synuclein",
  "term_label": "synaptic vesicle transport",
  "term_id": "GO:0048489"
}